{
  "term_id": "GO:0006357",
  "gene_symbol": "ZNF441",
  "gene": "UniProtKB:Q8N8Z8",
  "term_label": "regulation of transcription by RNA polymerase II",
  "gene_name": "Zinc finger protein 441"
}